{
  "term_label": "intracellular signal transduction",
  "term_id": "GO:0035556",
  "gene_name": "Nucleotide-binding oligomerization domain-containing protein 2",
  "gene_symbol": "NOD2",
  "gene": "UniProtKB:Q9HC29"
}